{
  "term_id": "GO:0008143",
  "gene": "UniProtKB:P29558",
  "term_label": "poly(A) binding",
  "gene_name": "RNA-binding motif, single-stranded-interacting protein 1",
  "gene_symbol": "RBMS1"
}